urea catabolic process [GO:0043419] (biological process) Sources: GOC:jl Relationships: is a type of urea metabolic process [GO:0019627]; is a type of amide catabolic process [GO:0043605]; is a type of GO:0044282 Also known as: urea breakdown, urea catabolism, urea decomposition, urea degradation Regulation: regulated by regulation of urea catabolic process [GO:0034254]; negatively regulated by GO:1901713; positively regulated by positive regulation of urea catabolic process [GO:1901714] Definition: The chemical reactions and pathways resulting in the breakdown of urea, the water soluble compound O=C-(NH2)2.